{
  "gene_name": "Centromere protein R",
  "gene": "UniProtKB:Q13352",
  "term_label": "Unknown biological process",
  "gene_symbol": "ITGB3BP",
  "term_id": "UNKNOWN:0002"
}